{
  "gene_symbol": "DDTL",
  "gene": "UniProtKB:A6NHG4",
  "term_id": "UNKNOWN:0002",
  "term_label": "Unknown biological process",
  "gene_name": "D-dopachrome decarboxylase-like protein"
}